{
  "term_id": "GO:0042765",
  "term_label": "GPI-anchor transamidase complex",
  "gene_symbol": "PIGU",
  "gene": "UniProtKB:Q9H490",
  "gene_name": "Phosphatidylinositol glycan anchor biosynthesis class U protein"
}